{
  "gene_name": "Ubiquitin carboxyl-terminal hydrolase 17-like protein 22",
  "term_label": "regulation of apoptotic process",
  "gene_symbol": "USP17L22",
  "term_id": "GO:0042981",
  "gene": "UniProtKB:D6RA61"
}